negative regulation of acrosome reaction [GO:1902225] (biological process) Relationships: is a type of regulation of acrosome reaction [GO:0060046]; is a type of negative regulation of reproductive process [GO:2000242]; negatively regulates acrosome reaction [GO:0007340] References: PMID:23430248 Sources: GOC:TermGenie Also known as: down regulation of acrosome reaction, down-regulation of acrosome reaction, downregulation of acrosome reaction, inhibition of acrosome reaction Definition: Any process that stops, prevents or reduces the frequency, rate or extent of acrosome reaction.